female sex differentiation [GO:0046660] (biological process) Definition: The establishment of the sex of a female organism by physical differentiation. Sources: GOC:bf Relationships: is a type of GO:0007548; is part of multicellular organism development [GO:0007275]